{
  "gene_name": "Colipase-like protein 1",
  "term_label": "enzyme activator activity",
  "gene_symbol": "CLPSL1",
  "gene": "UniProtKB:A2RUU4",
  "term_id": "GO:0008047"
}